{
  "gene_name": "Nucleotide sugar transporter SLC35B4",
  "term_label": "UDP-N-acetylglucosamine transmembrane transport",
  "gene_symbol": "SLC35B4",
  "term_id": "GO:1990569",
  "gene": "UniProtKB:Q969S0"
}